oligoxyloglucan beta-glycosidase activity [GO:0033935] (molecular function) Also known as: isoprimeverose-producing oligoxyloglucan hydrolase activity, oligoxyloglucan hydrolase activity, oligoxyloglucan xyloglucohydrolase activity Sources: EC:3.2.1.120 Relationships: is_a beta-glucosidase activity [GO:0008422] Definition: Catalysis of the hydrolysis of (1->4)-beta-D-glucosidic links in oligoxyloglucans so as to remove successive isoprimeverose (i.e. alpha-xylo-1,6-beta-D-glucosyl-) residues from the non-reducing chain ends.